{
  "term_label": "Unknown cellular component",
  "gene_symbol": "FDCSP",
  "gene": "UniProtKB:Q8NFU4",
  "gene_name": "Follicular dendritic cell secreted peptide",
  "term_id": "UNKNOWN:0003"
}